{
  "gene_symbol": "TRMT2B",
  "gene_name": "tRNA (uracil-5-)-methyltransferase homolog B",
  "term_id": "UNKNOWN:0001",
  "term_label": "Unknown molecular function",
  "gene": "UniProtKB:Q96GJ1"
}